{
  "gene": "UniProtKB:Q9UJV9",
  "term_id": "GO:0003724",
  "gene_name": "Probable ATP-dependent RNA helicase DDX41",
  "term_label": "RNA helicase activity",
  "gene_symbol": "DDX41"
}